{
  "term_id": "GO:0032355",
  "gene": "UniProtKB:P47710",
  "gene_name": "Alpha-S1-casein",
  "gene_symbol": "CSN1S1",
  "term_label": "response to estradiol"
}